{
  "gene_name": "Proteasome inhibitor PI31 subunit",
  "gene_symbol": "PSMF1",
  "term_label": "ubiquitin-dependent protein catabolic process",
  "gene": "UniProtKB:Q92530",
  "term_id": "GO:0006511"
}